negative regulation of natural killer cell differentiation involved in immune response [GO:0032827] (biological process) Definition: Any process that stops, prevents, or reduces the frequency, rate or extent of natural killer cell differentiation as part of an immune response. Note: Note that immunologists typically use the word 'development' to refer to cells of B or T cell lineages undergoing the process that GO describes as 'cell differentiation'. Also known as: inhibition of natural killer cell differentiation during immune response, down regulation of natural killer cell differentiation during immune response, down-regulation of natural killer cell differentiation during immune response, downregulation of natural killer cell differentiation during immune response, negative regulation of NK cell differentiation during immune response, negative regulation of natural killer cell development involved in immune response, negative regulation of natural killer cell differentiation during immune response Sources: GOC:mah Relationships: is a type of negative regulation of immune effector process [GO:0002698]; is a type of GO:0032824; is_a regulation of natural killer cell differentiation involved in immune response [GO:0032826]; is a type of GO:0050777; negatively regulates natural killer cell differentiation involved in immune response [GO:0002325]